vesicle fusion with nuclear membrane involved in mitotic nuclear envelope reassembly [GO:0007086] (biological process) Definition: The cell cycle process that results in the joining of the lipid bilayer membrane around a vesicle with the lipid bilayer membrane around the nucleus, and contributes to mitotic nuclear envelope reassembly. Sources: GOC:jid, GOC:mah Relationships: is a type of GO:0000740; is a type of vesicle fusion [GO:0006906]; is a type of mitotic nuclear membrane organization [GO:0101024]; is part of mitotic nuclear membrane reassembly [GO:0007084]